{
  "gene_symbol": "SPACA4",
  "gene_name": "Sperm acrosome membrane-associated protein 4",
  "term_id": "GO:0016020",
  "gene": "UniProtKB:Q8TDM5",
  "term_label": "membrane"
}